oxidoreductase activity, acting on the CH-OH group of donors, NAD or NADP as acceptor [GO:0016616] (molecular function) Subtypes: acylglycerone-phosphate reductase (NADP+) activity [GO:0000140], (R,R)-butanediol dehydrogenase activity [GO:0000721], (3S)-3-hydroxyacyl-CoA dehydrogenase (NAD+) activity [GO:0003857], GO:0003858, 3-isopropylmalate dehydrogenase activity [GO:0003862], IMP dehydrogenase activity [GO:0003938], UDP-glucose 6-dehydrogenase activity [GO:0003979], 3-oxoacyl-[acyl-carrier-protein] reductase (NADPH) activity [GO:0004316], glucose-6-phosphate dehydrogenase activity [GO:0004345], GO:0004399, homoserine dehydrogenase activity [GO:0004412], hydroxymethylglutaryl-CoA reductase (NADPH) activity [GO:0004420], GO:0004448, ketol-acid reductoisomerase activity [GO:0004455], malate dehydrogenase (decarboxylating) (NAD+) activity [GO:0004471], GO:0004473, GO:0004616, phosphoglycerate dehydrogenase activity [GO:0004617], sepiapterin reductase (NADP+) activity [GO:0004757], shikimate 3-dehydrogenase (NADP+) activity [GO:0004764], phosphogluconate 2-dehydrogenase activity [GO:0008114], GO:0008442, 2-dehydropantoate 2-reductase activity [GO:0008677], 2-deoxy-D-gluconate 3-dehydrogenase activity [GO:0008678], 2-hydroxy-3-oxopropionate reductase activity [GO:0008679], 3-hydroxybutyryl-CoA dehydrogenase activity [GO:0008691], GO:0008703, GO:0008743, GO:0008762, GO:0008831, fructuronate reductase activity [GO:0008866], galactitol-1-phosphate 5-dehydrogenase activity [GO:0008868], gluconate dehydrogenase activity [GO:0008875], glycerol dehydrogenase (NAD+) activity [GO:0008888], lactaldehyde reductase activity [GO:0008912], mannitol-1-phosphate 5-dehydrogenase activity [GO:0008926], sorbitol-6-phosphate 2-dehydrogenase activity [GO:0009010], tagaturonate reductase activity [GO:0009026], tartrate dehydrogenase activity [GO:0009027], ureidoglycolate dehydrogenase activity [GO:0009040], L-galactose dehydrogenase activity [GO:0010349], UDP-4-keto-rhamnose-4-keto-reductase activity [GO:0010490], GO:0016404, GO:0016617, hydroxypyruvate reductase [NAD(P)H] activity [GO:0016618], 5-exo-hydroxycamphor dehydrogenase activity [GO:0018452], GO:0018454, alcohol dehydrogenase [NAD(P)+] activity [GO:0018455], isopiperitenol dehydrogenase activity [GO:0018458], GO:0018459, cyclohexanol dehydrogenase activity [GO:0018460], fluoren-9-ol dehydrogenase activity [GO:0018461], GO:0018462, GO:0018463, 3-hydroxypimeloyl-CoA dehydrogenase activity [GO:0018464], (R)-aminopropanol dehydrogenase activity [GO:0019147], galactose 1-dehydrogenase activity [GO:0019151], acetoin dehydrogenase (NAD+) activity [GO:0019152], GO:0019155, methylglyoxal reductase (NADH) activity [GO:0019170], L-malate dehydrogenase (NAD+) activity [GO:0030060], quinate 3-dehydrogenase (NAD+) activity [GO:0030266], 1-deoxy-D-xylulose-5-phosphate reductoisomerase activity [GO:0030604], serine 3-dehydrogenase activity [GO:0031132], sorbose reductase activity [GO:0032115], phenylcoumaran benzylic ether reductase activity [GO:0032442], dTDP-galactose 6-dehydrogenase activity [GO:0033701], (+)-trans-carveol dehydrogenase activity [GO:0033702], GO:0033705, 3''-deamino-3''-oxonicotianamine reductase activity [GO:0033707], isocitrate-homoisocitrate dehydrogenase activity [GO:0033708], D-arabinitol dehydrogenase (NADP+) activity [GO:0033709], 4-phosphoerythronate dehydrogenase activity [GO:0033711], 1,5-anhydro-D-fructose reductase (1,5-anhydro-D-mannitol-forming) activity [GO:0033712], steroid dehydrogenase activity, acting on the CH-OH group of donors, NAD or NADP as acceptor [GO:0033764], hydroxymethylfurfural reductase activity [GO:0033790], GO:0033792, hydroxymethylfurfural reductase (NADH) activity [GO:0033833], hydroxymethylfurfural reductase (NADPH) activity [GO:0033845], GO:0034256, very long-chain-3-hydroxyacyl-CoA dehydrogenase activity [GO:0035380], GO:0035527, prostaglandin H2 endoperoxidase reductase activity [GO:0036130], GO:0036131, GO:0036185, GO:0036354, 2-dehydropantolactone reductase activity [GO:0036441], GO:0042356, GO:0043713, 2-hydroxymethylglutarate dehydrogenase activity [GO:0043718], methylglyoxal reductase (NADPH) activity [GO:0043892], GO:0044103, GO:0044105, GO:0045290, 6-endo-hydroxycineole dehydrogenase activity [GO:0045481], cinnamyl-alcohol dehydrogenase activity [GO:0045551], dihydroflavanol 4-reductase activity [GO:0045552], mannitol dehydrogenase activity [GO:0046029], GO:0046526, D-malate dehydrogenase (decarboxylating) (NAD+) activity [GO:0046553], L-malate dehydrogenase (NADP+) activity [GO:0046554], GO:0046998, 2-dehydro-3-deoxy-D-gluconate 6-dehydrogenase activity [GO:0047000], 2-dehydro-3-deoxy-D-gluconate 5-dehydrogenase activity [GO:0047001], L-arabinitol 2-dehydrogenase activity [GO:0047002], GO:0047003, UDP-N-acetylglucosamine 6-dehydrogenase activity [GO:0047004], 3-alpha-hydroxy-5-beta-androstane-17-one 3-alpha-dehydrogenase activity [GO:0047009], GO:0047010, glycerol-3-phosphate 1-dehydrogenase (NADP+) activity [GO:0047014], 3-hydroxy-2-methylbutyryl-CoA dehydrogenase activity [GO:0047015], cholest-5-ene-3-beta,7-alpha-diol 3-beta-dehydrogenase activity [GO:0047016], prostaglandin F synthase activity [GO:0047017], indole-3-acetaldehyde reductase (NADPH) activity [GO:0047019], 15-hydroxyprostaglandin-D dehydrogenase (NADP+) activity [GO:0047020], 15-hydroxyprostaglandin dehydrogenase (NADP+) activity [GO:0047021], 3-oxoacyl-[acyl-carrier-protein] reductase (NADH) activity [GO:0047025], benzyl-2-methyl-hydroxybutyrate dehydrogenase activity [GO:0047027], 6-pyruvoyltetrahydropterin 2'-reductase activity [GO:0047028], (R)-4-hydroxyphenyllactate dehydrogenase (NADP+) activity [GO:0047029], 4-hydroxycyclohexanecarboxylate dehydrogenase activity [GO:0047030], diethyl 2-methyl-3-oxosuccinate reductase activity [GO:0047031], 3-alpha-hydroxyglycyrrhetinate dehydrogenase activity [GO:0047032], 15-hydroxyprostaglandin-I dehydrogenase (NADP+) activity [GO:0047033], 15-hydroxyicosatetraenoate dehydrogenase activity [GO:0047034], codeinone reductase (NADPH) activity [GO:0047036], salutaridine reductase (NADPH) activity [GO:0047037], D-arabinitol 2-dehydrogenase activity [GO:0047038], tetrahydroxynaphthalene reductase activity [GO:0047039], (S)-carnitine 3-dehydrogenase activity [GO:0047041], GO:0047043, homoisocitrate dehydrogenase activity [GO:0047046], oxaloglycolate reductase (decarboxylating) activity [GO:0047047], 3-hydroxybenzyl-alcohol dehydrogenase activity [GO:0047048], GO:0047049, GO:0047050, (R)-3-hydroxyacid-ester dehydrogenase activity [GO:0047108], (S)-3-hydroxyacid-ester dehydrogenase activity [GO:0047109], (+)-borneol dehydrogenase activity [GO:0047500], (+)-neomenthol dehydrogenase activity [GO:0047501], (+)-sabinol dehydrogenase activity [GO:0047502], (-)-borneol dehydrogenase activity [GO:0047503], (-)-menthol dehydrogenase activity [GO:0047504], (S,S)-butanediol dehydrogenase activity [GO:0047512], 1,3-propanediol dehydrogenase activity [GO:0047516], GO:0047535, 2-oxoadipate reductase activity [GO:0047550], 3-dehydro-L-gulonate 2-dehydrogenase activity [GO:0047559], GO:0047560, 3-hydroxypropionate dehydrogenase (NAD+) activity [GO:0047565], 4-hydroxybutyrate dehydrogenase activity [GO:0047577], 8-oxocoformycin reductase activity [GO:0047599], aldose 1-dehydrogenase activity [GO:0047640], aldose-6-phosphate reductase (NADPH) activity [GO:0047641], allyl-alcohol dehydrogenase activity [GO:0047655], apiose 1-reductase activity [GO:0047674], aryl-alcohol dehydrogenase (NADP+) activity [GO:0047681], galactitol 2-dehydrogenase activity [GO:0047713], indanol dehydrogenase activity [GO:0047718], indolelactate dehydrogenase (NAD+) activity [GO:0047722], carnitine 3-dehydrogenase activity [GO:0047728], chlordecone reductase activity [GO:0047743], cyclohexane-1,2-diol dehydrogenase activity [GO:0047795], D-arabinitol 4-dehydrogenase activity [GO:0047813], D-iditol 2-dehydrogenase activity [GO:0047824], GO:0047832, D-threo-aldose 1-dehydrogenase activity [GO:0047834], D-xylose 1-dehydrogenase (NADP+) activity [GO:0047837], D-xylose 1-dehydrogenase (NAD+) activity [GO:0047838], dihydrobunolol dehydrogenase activity [GO:0047855], diiodophenylpyruvate reductase (NAD+) activity [GO:0047860], dimethylmalate dehydrogenase activity [GO:0047867], erythrulose reductase activity [GO:0047880], GO:0047886, GO:0047890, fructose 5-dehydrogenase (NADP+) activity [GO:0047903], galactose 1-dehydrogenase (NADP+) activity [GO:0047910], GDP-6-deoxy-D-talose 4-dehydrogenase activity [GO:0047916], GDP-mannose 6-dehydrogenase activity [GO:0047919], geraniol dehydrogenase activity [GO:0047924], GO:0047936, L-glucuronate reductase activity [GO:0047939], glucuronolactone reductase activity [GO:0047941], glycerol-3-phosphate dehydrogenase [NAD(P)+] activity [GO:0047952], glycerol 2-dehydrogenase (NADP+) activity [GO:0047953], glycerol dehydrogenase (NADP+) activity [GO:0047956], hydroxymalonate dehydrogenase activity [GO:0047993], 3-ketoglucose-reductase activity [GO:0048258], isopropanol dehydrogenase (NADP+) activity [GO:0050009], L-arabinitol 4-dehydrogenase activity [GO:0050019], L-arabinose 1-dehydrogenase (NAD+) activity [GO:0050022], L-glycol dehydrogenase activity [GO:0050026], GO:0050034, L-threonate 3-dehydrogenase activity [GO:0050036], L-xylose 1-dehydrogenase activity [GO:0050037], GO:0050038, GO:0050039, GO:0050060, GO:0050085, GO:0050086, GO:0050088, GO:0050090, GO:0050104, morphine 6-dehydrogenase activity [GO:0050109], N-acetylhexosamine 1-dehydrogenase activity [GO:0050120], N-acylmannosamine 1-dehydrogenase activity [GO:0050123], omega-hydroxydecanoate dehydrogenase activity [GO:0050153], pantoate 4-dehydrogenase activity [GO:0050166], propanediol-phosphate dehydrogenase activity [GO:0050216], prostaglandin E2 9-reductase activity [GO:0050221], pyridoxal 4-dehydrogenase activity [GO:0050235], GO:0050255, ribitol-5-phosphate 2-dehydrogenase [NAD(P)+] activity [GO:0050256], ribose 1-dehydrogenase (NADP+) activity [GO:0050259], GO:0050268, sequoyitol dehydrogenase activity [GO:0050280], GO:0050287, tropine dehydrogenase activity [GO:0050356], GO:0050358, GO:0050388, vomifoliol 4'-dehydrogenase activity [GO:0050396], sulcatone reductase activity [GO:0050491], glycerol-1-phosphate dehydrogenase [NAD(P)+] activity [GO:0050492], 4-hydroxythreonine-4-phosphate dehydrogenase activity [GO:0050570], GO:0050571, GO:0050572, dTDP-4-dehydro-6-deoxyglucose reductase activity [GO:0050573], 2-(R)-hydroxypropyl-CoM dehydrogenase activity [GO:0050574], 2-(S)-hydroxypropyl-CoM dehydrogenase activity [GO:0050575], GDP-L-fucose synthase activity [GO:0050577], (2R)-2-hydroxyacid dehydrogenase (NADP+) activity [GO:0050578], vellosimine dehydrogenase activity [GO:0050579], GO:0050580, 4-carboxy-2-hydroxymuconate semialdehyde hemiacetal dehydrogenase activity [GO:0050606], S-(hydroxymethyl)glutathione dehydrogenase [NAD(P)+] activity [GO:0051903], quinate 3-dehydrogenase (NADP+) activity [GO:0052733], shikimate 3-dehydrogenase (NAD+) activity [GO:0052734], cyclopentanol dehydrogenase activity [GO:0055041], 3-sulfolactaldehyde reductase activity [GO:0061596], S-nitrosoglutathione reductase (NADH) activity [GO:0080007], UDP-N-acetyl-D-mannosamine dehydrogenase activity [GO:0089714], 5(S)-hydroxyeicosatetraenoic acid dehydrogenase activity [GO:0097265], UDP-glucuronate dehydrogenase activity [GO:0099618], zerumbone synthase activity [GO:0102069], GO:0102098, S-sulfolactate dehydrogenase activity [GO:0102155], (R)-sulfopropanediol 2-dehydrogenase activity [GO:0102157], GO:0102311, GO:0102357, phenylacetaldehyde reductase activity [GO:0102386], GO:0102394, L-2-hydroxycarboxylate dehydrogenase (NAD+) activity [GO:0102443], scyllo-inositol dehydrogenase (NADP+) activity [GO:0102497], D-fructuronate reductase activity [GO:0102501], UDP-N-acetyl-alpha-D-quinovosamine dehydrogenase activity [GO:0102538], UDP-N-acetyl-alpha-D-fucosamine dehydrogenase activity [GO:0102539], GO:0102635, (R)-lactaldehyde dehydrogenase activity [GO:0102641], momilactone-A synthase [NAD(P)H] activity [GO:0102960], 10-hydroxygeraniol oxidoreductase activity [GO:0102967], 10-hydroxygeranial oxidoreductase activity [GO:0102968], 10-oxogeraniol oxidoreductase activity [GO:0102969], hydroxyversicolorone reductase activity [GO:0102974], versiconal hemiacetal acetate reductase activity [GO:0102975], versiconal reductase activity [GO:0102976], UDP-3-dehydro-alpha-D-glucose dehydrogenase activity [GO:0102982], GO:0103002, L-glyceraldehyde 3-phosphate reductase activity [GO:0103037], glucose-6-phosphate 3-dehydrogenase activity [GO:0103074], glyoxylate reductase activity [GO:0106345], (3R)-3-hydroxyacyl-CoA dehydrogenase (NAD+) activity [GO:0106386], GO:0120529, (R)-2-hydroxyglutarate (NAD+) dehydrogenase activity [GO:0120568], GO:0140175, 5'-hydroxyaverantin dehydrogenase activity [GO:0140396], hydroxymethylglutaryl-CoA reductase (NADH) activity [GO:0140643], GO:0140860, GO:0141040, S-nitrosoglutathione reductase (NADPH) activity [GO:0160163], cardiolipin dehydrogenase (NAD+) activity [GO:0160241], phosphatidylglycerol dehydrogenase (NAD+) activity [GO:0160242], GO:1990002 Definition: Catalysis of an oxidation-reduction (redox) reaction in which a CH-OH group acts as a hydrogen or electron donor and reduces NAD+ or NADP. Relationships: is a type of oxidoreductase activity, acting on CH-OH group of donors [GO:0016614] Sources: EC:1.1.1.-